{
  "term_id": "UNKNOWN:0002",
  "term_label": "Unknown biological process",
  "gene_name": "Small cysteine and glycine repeat-containing protein 10",
  "gene_symbol": "SCYGR10",
  "gene": "UniProtKB:A0A286YEX9"
}